{
  "term_id": "GO:0002080",
  "gene_name": "Coiled-coil domain-containing protein 136",
  "term_label": "acrosomal membrane",
  "gene_symbol": "CCDC136",
  "gene": "UniProtKB:Q96JN2"
}